{
  "term_id": "GO:0005634",
  "term_label": "nucleus",
  "gene_symbol": "ZGRF1",
  "gene_name": "Protein ZGRF1",
  "gene": "UniProtKB:Q86YA3"
}